negative regulation of extracellular matrix organization [GO:1903054] (biological process) References: PMID:22357537 Sources: GOC:BHF, GOC:TermGenie, GOC:rl, GO_REF:0000058 Also known as: down regulation of extracellular matrix organisation, down regulation of extracellular matrix organization, down-regulation of extracellular matrix organisation, down-regulation of extracellular matrix organization, downregulation of extracellular matrix organisation, downregulation of extracellular matrix organization, negative regulation of extracellular matrix organisation, inhibition of extracellular matrix organisation, inhibition of extracellular matrix organization, down regulation of extracellular matrix organization and biogenesis, down-regulation of extracellular matrix organization and biogenesis, downregulation of extracellular matrix organization and biogenesis, inhibition of extracellular matrix organization and biogenesis, negative regulation of extracellular matrix organization and biogenesis Subtypes: GO:0003332, negative regulation of extracellular matrix disassembly [GO:0010716], negative regulation of extracellular matrix assembly [GO:1901202], negative regulation of collagen fibril organization [GO:1904027] Definition: Any process that stops, prevents or reduces the frequency, rate or extent of extracellular matrix organization. Relationships: is a type of negative regulation of cellular component organization [GO:0051129]; is a type of regulation of extracellular matrix organization [GO:1903053]; negatively regulates extracellular matrix organization [GO:0030198]